{
  "term_label": "Unknown cellular component",
  "gene": "UniProtKB:A6NKG5",
  "gene_name": "Retrotransposon-like protein 1",
  "gene_symbol": "RTL1",
  "term_id": "UNKNOWN:0003"
}